{
  "term_label": "nucleus",
  "gene": "UniProtKB:P52292",
  "term_id": "GO:0005634",
  "gene_name": "Importin subunit alpha-1",
  "gene_symbol": "KPNA2"
}